{
  "term_id": "GO:0000978",
  "gene": "UniProtKB:Q8IWY8",
  "gene_symbol": "ZSCAN29",
  "term_label": "RNA polymerase II cis-regulatory region sequence-specific DNA binding",
  "gene_name": "Zinc finger and SCAN domain-containing protein 29"
}